sensory perception of sound [GO:0007605] (biological process) Definition: The series of events required for an organism to receive an auditory stimulus, convert it to a molecular signal, and recognize and characterize the signal. Sonic stimuli are detected in the form of vibrations and are processed to form a sound. Also known as: hearing, perception of sound Sources: GOC:ai Relationships: is a type of GO:0050954